{
  "gene_name": "Olfactory receptor 13F1",
  "term_label": "detection of chemical stimulus involved in sensory perception of smell",
  "gene": "UniProtKB:Q8NGS4",
  "gene_symbol": "OR13F1",
  "term_id": "GO:0050911"
}